{
  "gene": "UniProtKB:Q6WCQ1",
  "gene_name": "Myosin phosphatase Rho-interacting protein",
  "term_label": "actin cytoskeleton",
  "term_id": "GO:0015629",
  "gene_symbol": "MPRIP"
}